glycerol dehydrogenase (NAD+) activity [GO:0008888] (molecular function) Sources: RHEA:13769 Also known as: glycerol dehydrogenase activity, NAD-linked glycerol dehydrogenase activity Definition: Catalysis of the reaction: glycerol + NAD+ = glycerone + H+ + NADH. Relationships: is_a oxidoreductase activity, acting on the CH-OH group of donors, NAD or NADP as acceptor [GO:0016616]